symbiont-mediated suppression of host immune response [GO:0052562] (BP) Definition: A process in which a symbiont interferes with, inhibits or disrupts the normal execution of an immune response of the host organism. The immune response is any immune system process that functions in the calibrated response of an organism to a potential internal or invasive threat. The host is defined as the larger of the organisms involved in a symbiotic interaction. Sources: GOC:mtg_pamgo_17jul06 Also known as: negative regulation by organism of immune response of other organism involved in symbiotic interaction, down regulation by symbiont of host immune response, down-regulation by symbiont of host immune response, downregulation by symbiont of host immune response, negative regulation by symbiont of host immune response, suppression by symbiont of host immune response, inhibition by symbiont of host immune response Relationships: is a type of symbiont-mediated perturbation of host immune response [GO:0052553] Subtypes: symbiont-mediated suppression of host adaptive immune response [GO:0039504], symbiont-mediated suppression of host innate immune response [GO:0052170], GO:0141140